{
  "gene_name": "Alpha-aminoadipic semialdehyde dehydrogenase",
  "gene": "UniProtKB:P49419",
  "term_id": "UNKNOWN:0002",
  "term_label": "Unknown biological process",
  "gene_symbol": "ALDH7A1"
}